positive regulation of tyrosine phosphorylation of STAT protein [GO:0042531] (BP) Relationships: is a type of regulation of tyrosine phosphorylation of STAT protein [GO:0042509]; is a type of positive regulation of peptidyl-tyrosine phosphorylation [GO:0050731]; positively regulates GO:0007260 Definition: Any process that activates or increases the frequency, rate or extent of the introduction of a phosphate group to a tyrosine residue of a STAT (Signal Transducer and Activator of Transcription) protein. References: PMID:11426647 Sources: GOC:jl Also known as: up regulation of tyrosine phosphorylation of STAT protein, up-regulation of tyrosine phosphorylation of STAT protein, upregulation of tyrosine phosphorylation of STAT protein, activation of tyrosine phosphorylation of STAT protein, activation of tyrosine phosphorylation of Stat1 protein, activation of tyrosine phosphorylation of Stat2 protein, activation of tyrosine phosphorylation of Stat3 protein, activation of tyrosine phosphorylation of Stat4 protein, activation of tyrosine phosphorylation of Stat5 protein, activation of tyrosine phosphorylation of Stat6 protein, activation of tyrosine phosphorylation of Stat7 protein, positive regulation of tyrosine phosphorylation of Stat1 protein, positive regulation of tyrosine phosphorylation of Stat2 protein, positive regulation of tyrosine phosphorylation of Stat3 protein, positive regulation of tyrosine phosphorylation of Stat4 protein, positive regulation of tyrosine phosphorylation of Stat5 protein, positive regulation of tyrosine phosphorylation of Stat6 protein, positive regulation of tyrosine phosphorylation of Stat7 protein, stimulation of tyrosine phosphorylation of STAT protein, stimulation of tyrosine phosphorylation of Stat1 protein, stimulation of tyrosine phosphorylation of Stat2 protein, stimulation of tyrosine phosphorylation of Stat3 protein, stimulation of tyrosine phosphorylation of Stat4 protein, stimulation of tyrosine phosphorylation of Stat5 protein, stimulation of tyrosine phosphorylation of Stat6 protein, stimulation of tyrosine phosphorylation of Stat7 protein, up regulation of tyrosine phosphorylation of Stat1 protein, up regulation of tyrosine phosphorylation of Stat2 protein, up regulation of tyrosine phosphorylation of Stat3 protein, up regulation of tyrosine phosphorylation of Stat4 protein, up regulation of tyrosine phosphorylation of Stat5 protein, up regulation of tyrosine phosphorylation of Stat6 protein, up regulation of tyrosine phosphorylation of Stat7 protein, up-regulation of tyrosine phosphorylation of Stat1 protein, up-regulation of tyrosine phosphorylation of Stat2 protein, up-regulation of tyrosine phosphorylation of Stat3 protein, up-regulation of tyrosine phosphorylation of Stat4 protein, up-regulation of tyrosine phosphorylation of Stat5 protein, up-regulation of tyrosine phosphorylation of Stat6 protein, up-regulation of tyrosine phosphorylation of Stat7 protein, upregulation of tyrosine phosphorylation of Stat1 protein, upregulation of tyrosine phosphorylation of Stat2 protein, upregulation of tyrosine phosphorylation of Stat3 protein, upregulation of tyrosine phosphorylation of Stat4 protein, upregulation of tyrosine phosphorylation of Stat5 protein, upregulation of tyrosine phosphorylation of Stat6 protein, upregulation of tyrosine phosphorylation of Stat7 protein